{
  "gene_symbol": "ZNF155",
  "gene_name": "Zinc finger protein 155",
  "term_id": "UNKNOWN:0001",
  "gene": "UniProtKB:Q12901",
  "term_label": "Unknown molecular function"
}